{
  "gene": "UniProtKB:Q9Y689",
  "term_label": "intracellular protein transport",
  "gene_symbol": "ARL5A",
  "term_id": "GO:0006886",
  "gene_name": "ADP-ribosylation factor-like protein 5A"
}